{
  "term_label": "RNA polymerase II cis-regulatory region sequence-specific DNA binding",
  "gene_name": "Zinc finger protein 736",
  "gene": "UniProtKB:B4DX44",
  "gene_symbol": "ZNF736",
  "term_id": "GO:0000978"
}